{
  "gene_name": "Homeobox protein Hox-A10",
  "term_label": "RNA polymerase II cis-regulatory region sequence-specific DNA binding",
  "term_id": "GO:0000978",
  "gene_symbol": "HOXA10",
  "gene": "UniProtKB:P31260"
}